{
  "term_label": "lysosome",
  "gene_name": "DNA damage-regulated autophagy modulator protein 1",
  "term_id": "GO:0005764",
  "gene_symbol": "DRAM1",
  "gene": "UniProtKB:Q8N682"
}